{
  "term_label": "Unknown cellular component",
  "term_id": "UNKNOWN:0003",
  "gene_name": "ADAMTS-like protein 5",
  "gene_symbol": "ADAMTSL5",
  "gene": "UniProtKB:Q6ZMM2"
}